{
  "gene_symbol": "UBL3",
  "term_id": "UNKNOWN:0001",
  "term_label": "Unknown molecular function",
  "gene": "UniProtKB:O95164",
  "gene_name": "Ubiquitin-like protein 3"
}